{
  "term_label": "proteasome regulatory particle, base subcomplex",
  "gene": "UniProtKB:Q13200",
  "gene_name": "26S proteasome non-ATPase regulatory subunit 2",
  "term_id": "GO:0008540",
  "gene_symbol": "PSMD2"
}